{
  "gene": "UniProtKB:P0CE67",
  "gene_symbol": "LINC02877",
  "term_label": "Unknown biological process",
  "term_id": "UNKNOWN:0002",
  "gene_name": "Putative uncharacterized protein encoded by LINC02877"
}